{
  "term_id": "GO:0045830",
  "gene_symbol": "SHLD1",
  "gene_name": "Shieldin complex subunit 1",
  "term_label": "positive regulation of isotype switching",
  "gene": "UniProtKB:Q8IYI0"
}